{
  "term_label": "fatty acid binding",
  "gene": "UniProtKB:Q15067",
  "gene_symbol": "ACOX1",
  "term_id": "GO:0005504",
  "gene_name": "Peroxisomal acyl-coenzyme A oxidase 1"
}